{
  "term_label": "DNA-templated transcription elongation",
  "gene_name": "AF4_FMR2 family member 1",
  "term_id": "GO:0006354",
  "gene_symbol": "AFF1",
  "gene": "UniProtKB:P51825"
}